{
  "gene_name": "Transcription factor YY2",
  "gene_symbol": "YY2",
  "term_id": "GO:0031519",
  "gene": "UniProtKB:O15391",
  "term_label": "PcG protein complex"
}